{
  "term_label": "morphogenesis of an epithelium",
  "term_id": "GO:0002009",
  "gene_symbol": "KRT24",
  "gene": "UniProtKB:Q2M2I5",
  "gene_name": "Keratin, type I cytoskeletal 24"
}